CD4-positive, alpha-beta T cell costimulation [GO:0035783] (biological process) Relationships: is a type of GO:0031295; is a type of positive regulation of CD4-positive, alpha-beta T cell activation [GO:2000516] Definition: The process of providing, via surface-bound receptor-ligand pairs, a second, antigen-independent, signal in addition to that provided by the T cell receptor to augment CD4-positive, alpha-beta T cell activation. Sources: CL:0000624, GOC:BHF, GOC:pr Regulation: regulated by regulation of CD4-positive, alpha-beta T cell costimulation [GO:1900279]; negatively regulated by negative regulation of CD4-positive, alpha-beta T cell costimulation [GO:1900280]; positively regulated by GO:1900281 Also known as: CD4-positive, alpha beta T cell costimulation